focal adhesion assembly [GO:0048041] (biological process) Regulation: regulated by regulation of focal adhesion assembly [GO:0051893]; positively regulated by positive regulation of focal adhesion assembly [GO:0051894]; negatively regulated by negative regulation of focal adhesion assembly [GO:0051895] Also known as: adhesion plaque assembly, focal adhesion formation Definition: The aggregation and bonding together of a set of components to form a focal adhesion, a complex of intracellular signaling and structural proteins that provides a structural link between the internal actin cytoskeleton and the ECM, and also function as a locus of signal transduction activity. Relationships: is a type of cell-substrate junction assembly [GO:0007044]; is part of cell-matrix adhesion [GO:0007160] Sources: GOC:jid, GOC:mah